{
  "gene_name": "Transmembrane protein 245",
  "term_label": "Unknown cellular component",
  "gene": "UniProtKB:Q9H330",
  "term_id": "UNKNOWN:0003",
  "gene_symbol": "TMEM245"
}